{
  "term_id": "GO:0000978",
  "gene": "UniProtKB:Q15475",
  "term_label": "RNA polymerase II cis-regulatory region sequence-specific DNA binding",
  "gene_symbol": "SIX1",
  "gene_name": "Homeobox protein SIX1"
}